{
  "gene_name": "Complex III assembly factor LYRM7",
  "term_label": "mitochondrial respiratory chain complex III assembly",
  "gene": "UniProtKB:Q5U5X0",
  "gene_symbol": "LYRM7",
  "term_id": "GO:0034551"
}